3 iron, 4 sulfur cluster binding [GO:0051538] (molecular function) Relationships: is_a GO:0051536 Also known as: 3 Fe 4 S cluster binding, 3 iron, 4 sulphur cluster binding, 3Fe-4S cluster binding, iron-sulfur cluster 3Fe-4S binding, iron-sulphur cluster 3Fe-4S binding, triiron tetrasulfide cluster binding, triiron tetrasulphide cluster binding References: PMID:15952888 Sources: GOC:ai, Wikipedia:Iron-sulfur_cluster Definition: Binding to a 3 iron, 4 sulfur (3Fe-4S) cluster; this cluster consists of three iron atoms, with the inorganic sulfur atoms found between the irons and acting as bridging ligands. It is essentially a 4Fe-4S cluster with one iron missing.